{
  "gene": "UniProtKB:Q13247",
  "gene_symbol": "SRSF6",
  "term_label": "regulation of alternative mRNA splicing, via spliceosome",
  "term_id": "GO:0000381",
  "gene_name": "Serine_arginine-rich splicing factor 6"
}